establishment of sister chromatid cohesion [GO:0034085] (biological process) Subtypes: establishment of mitotic sister chromatid cohesion [GO:0034087], establishment of meiotic sister chromatid cohesion [GO:0034089] References: PMID:14623866 Sources: GOC:jh, GOC:mah Definition: The process in which the sister chromatids of a replicated chromosome become associated with each other during S phase. Relationships: is a type of cell cycle process [GO:0022402]; is part of sister chromatid cohesion [GO:0007062]